{
  "gene_symbol": "DRGX",
  "gene": "UniProtKB:A6NNA5",
  "term_id": "GO:0000977",
  "term_label": "RNA polymerase II transcription regulatory region sequence-specific DNA binding",
  "gene_name": "Dorsal root ganglia homeobox protein"
}